{
  "gene_symbol": "CYP4F8",
  "term_id": "GO:0019369",
  "gene": "UniProtKB:P98187",
  "term_label": "arachidonate metabolic process",
  "gene_name": "Cytochrome P450 4F8"
}